{
  "gene_name": "Zinc finger protein 609",
  "gene": "UniProtKB:O15014",
  "gene_symbol": "ZNF609",
  "term_label": "Unknown molecular function",
  "term_id": "UNKNOWN:0001"
}